{
  "gene_name": "Sia-alpha-2,3-Gal-beta-1,4-GlcNAc-R:alpha 2,8-sialyltransferase",
  "term_label": "Unknown cellular component",
  "gene": "UniProtKB:O43173",
  "gene_symbol": "ST8SIA3",
  "term_id": "UNKNOWN:0003"
}